{
  "gene_name": "Protein argonaute-2",
  "gene": "UniProtKB:Q9UKV8",
  "term_label": "pre-miRNA processing",
  "term_id": "GO:0031054",
  "gene_symbol": "AGO2"
}